{
  "gene_name": "Neuronal cell adhesion molecule",
  "term_label": "plasma membrane",
  "gene": "UniProtKB:Q92823",
  "term_id": "GO:0005886",
  "gene_symbol": "NRCAM"
}